positive regulation of tolerance induction to nonself antigen [GO:0002657] (biological process) Sources: GOC:add Also known as: up regulation of tolerance induction to nonself antigen, up-regulation of tolerance induction to nonself antigen, upregulation of tolerance induction to nonself antigen, activation of tolerance induction to nonself antigen, stimulation of tolerance induction to nonself antigen Relationships: is a type of GO:0002654; is a type of regulation of tolerance induction to nonself antigen [GO:0002655]; positively regulates GO:0002462 Definition: Any process that activates or increases the frequency, rate, or extent of tolerance induction to nonself antigen.